{
  "term_id": "GO:0009897",
  "term_label": "external side of plasma membrane",
  "gene_symbol": "IZUMO1R",
  "gene_name": "Sperm-egg fusion protein Juno",
  "gene": "UniProtKB:A6ND01"
}